positive regulation of macrophage apoptotic process [GO:2000111] (biological process) Also known as: positive regulation of macrophage apoptosis, positive regulation of AICD, positive regulation of activation-induced cell death Sources: GOC:BHF, GOC:mtg_apoptosis Definition: Any process that activates or increases the frequency, rate or extent of macrophage apoptotic process. Relationships: is a type of positive regulation of myeloid cell apoptotic process [GO:0033034]; is a type of positive regulation of leukocyte apoptotic process [GO:2000108]; is a type of regulation of macrophage apoptotic process [GO:2000109]; positively regulates macrophage apoptotic process [GO:0071888]